{
  "term_id": "UNKNOWN:0002",
  "gene_name": "Thymosin beta 15B",
  "gene_symbol": "TMSB15B",
  "gene": "UniProtKB:A0A087X1C1",
  "term_label": "Unknown biological process"
}